{
  "gene": "UniProtKB:A6NH13",
  "term_id": "UNKNOWN:0003",
  "term_label": "Unknown cellular component",
  "gene_symbol": "DNAJC9-AS1",
  "gene_name": "Putative uncharacterized protein DNAJC9-AS1"
}